uracil binding [GO:0002058] (molecular function) Sources: GOC:hjd Relationships: is a type of pyrimidine nucleobase binding [GO:0002061] Definition: Binding to uracil.